regulation of toll-like receptor 11 signaling pathway [GO:0034171] (biological process) Also known as: regulation of TLR11 signaling pathway, regulation of toll-like receptor 11 signalling pathway References: PMID:16551253, PMID:17328678 Sources: GOC:add Definition: Any process that modulates the frequency, rate, or extent of toll-like receptor 11 signaling pathway. Subtypes: negative regulation of toll-like receptor 11 signaling pathway [GO:0034172], positive regulation of toll-like receptor 11 signaling pathway [GO:0034173] Relationships: is_a GO:0039531; regulates GO:0034170